{
  "gene_symbol": "NPIPB8",
  "term_id": "UNKNOWN:0001",
  "term_label": "Unknown molecular function",
  "gene": "UniProtKB:E9PQR5",
  "gene_name": "Nuclear pore complex-interacting protein family member B8"
}